thyroid hormone transport [GO:0070327] (biological process) Definition: The directed movement of thyroid hormone into, out of or within a cell, or between cells, by means of some agent such as a transporter or pore. Also known as: thyroxine transport, triiodothyronine transport Sources: GOC:rph Relationships: is a type of GO:0009914